regulation of sodium-dependent phosphate transport [GO:2000118] (biological process) Relationships: is a type of GO:0010966; regulates sodium-dependent phosphate transport [GO:0044341] Subtypes: GO:2000119, GO:2000120 Sources: GOC:BHF Definition: Any process that modulates the frequency, rate or extent of sodium-dependent phosphate transport.